{
  "term_id": "GO:0072659",
  "gene_symbol": "EFR3A",
  "term_label": "protein localization to plasma membrane",
  "gene": "UniProtKB:Q14156",
  "gene_name": "Protein EFR3 homolog A"
}